{
  "gene_name": "Succinate--CoA ligase [ADP-forming] subunit beta, mitochondrial",
  "term_id": "GO:0042709",
  "term_label": "succinate-CoA ligase complex",
  "gene_symbol": "SUCLA2",
  "gene": "UniProtKB:Q9P2R7"
}